{
  "term_id": "GO:0000086",
  "gene": "UniProtKB:P24941",
  "term_label": "G2/M transition of mitotic cell cycle",
  "gene_symbol": "CDK2",
  "gene_name": "Cyclin-dependent kinase 2"
}